inositol-1,3,4,5-tetrakisphosphate 6-kinase activity [GO:0000825] (molecular function) Sources: MetaCyc:RXN-7184 Definition: Catalysis of the reaction: 1D-myo-inositol 1,3,4,5-tetrakisphosphate + ATP = 1D-myo-inositol 1,3,4,5,6-pentakisphosphate + ADP + H+. Relationships: is a type of GO:0051765 Also known as: 1D-myo-inositol-tetrakisphosphate 6-kinase activity, inositol tetrakisphosphate 6-kinase activity, inositol 1,3,4,5-tetrakisphosphate 6-kinase activity